{
  "term_id": "GO:0005524",
  "term_label": "ATP binding",
  "gene": "UniProtKB:O14678",
  "gene_symbol": "ABCD4",
  "gene_name": "Lysosomal cobalamin transporter ABCD4"
}